{
  "term_label": "respiratory chain complex I",
  "term_id": "GO:0045271",
  "gene_symbol": "NDUFB6",
  "gene_name": "NADH dehydrogenase [ubiquinone] 1 beta subcomplex subunit 6",
  "gene": "UniProtKB:O95139"
}